{
  "term_id": "GO:0002040",
  "gene_name": "Lysyl oxidase homolog 2",
  "gene": "UniProtKB:Q9Y4K0",
  "term_label": "sprouting angiogenesis",
  "gene_symbol": "LOXL2"
}